{
  "gene": "UniProtKB:Q9ULI0",
  "gene_name": "ATPase family AAA domain-containing protein 2B",
  "term_label": "nucleosome disassembly",
  "gene_symbol": "ATAD2B",
  "term_id": "GO:0006337"
}